{
  "gene_symbol": "ZRANB3",
  "gene": "UniProtKB:Q5FWF4",
  "term_id": "GO:0043596",
  "term_label": "nuclear replication fork",
  "gene_name": "DNA annealing helicase and endonuclease ZRANB3"
}